{
  "term_label": "cell fate commitment",
  "term_id": "GO:0045165",
  "gene_name": "Protein Wnt-2b",
  "gene": "UniProtKB:Q93097",
  "gene_symbol": "WNT2B"
}